negative regulation of chondrocyte proliferation [GO:1902731] (biological process) Definition: Any process that stops, prevents, or reduces the frequency, rate or extent of the multiplication or reproduction of chondrocytes by cell division, resulting in the expansion of their population. A chondrocyte is a polymorphic cell that forms cartilage. References: PMID:23212449 Sources: GOC:TermGenie, GO_REF:0000058 Also known as: down regulation of cartilage cell proliferation, down regulation of chondrocyte cell proliferation, down regulation of chondrocyte proliferation, down-regulation of cartilage cell proliferation, down-regulation of chondrocyte cell proliferation, down-regulation of chondrocyte proliferation, downregulation of cartilage cell proliferation, downregulation of chondrocyte cell proliferation, downregulation of chondrocyte proliferation, negative regulation of cartilage cell proliferation, negative regulation of chondrocyte cell proliferation, inhibition of cartilage cell proliferation, inhibition of chondrocyte cell proliferation, inhibition of chondrocyte proliferation Relationships: is a type of negative regulation of cell population proliferation [GO:0008285]; negatively regulates GO:0035988